{
  "term_label": "Unknown cellular component",
  "term_id": "UNKNOWN:0003",
  "gene_symbol": "YAP1",
  "gene": "UniProtKB:P46937",
  "gene_name": "Transcriptional coactivator YAP1"
}